{
  "gene_symbol": "CA6",
  "gene": "UniProtKB:P23280",
  "term_label": "Unknown biological process",
  "gene_name": "Carbonic anhydrase 6",
  "term_id": "UNKNOWN:0002"
}